{
  "term_id": "GO:0043149",
  "gene_symbol": "FAM171A1",
  "gene_name": "Protein FAM171A1",
  "term_label": "stress fiber assembly",
  "gene": "UniProtKB:Q5VUB5"
}